{
  "gene": "UniProtKB:Q96MT7",
  "gene_name": "Cilia- and flagella-associated protein 44",
  "gene_symbol": "CFAP44",
  "term_label": "axoneme",
  "term_id": "GO:0005930"
}